{
  "gene_name": "TAF6-like RNA polymerase II p300_CBP-associated factor-associated factor 65 kDa subunit 6L",
  "term_label": "Unknown cellular component",
  "gene_symbol": "TAF6L",
  "term_id": "UNKNOWN:0003",
  "gene": "UniProtKB:Q9Y6J9"
}